{
  "term_id": "GO:0005764",
  "gene_symbol": "RRAGB",
  "gene_name": "Ras-related GTP-binding protein B",
  "term_label": "lysosome",
  "gene": "UniProtKB:Q5VZM2"
}